symbiont-mediated disruption of host cell-cell adhesion [GO:0141023] (biological process) Definition: A process in which a symbiont alters or subverts host cell adhesion ito its extracellular matrix. The host is defined as the larger of the organisms involved in a symbiotic interaction. Sources: GOC:curators Also known as: disruption by symbiont of host cell-cell adhesion Relationships: is a type of symbiont-mediated perturbation of host cellular process [GO:0044068]